{
  "term_label": "defense response to virus",
  "term_id": "GO:0051607",
  "gene": "UniProtKB:P20591",
  "gene_name": "Interferon-induced GTP-binding protein Mx1",
  "gene_symbol": "MX1"
}